{
  "gene_name": "Protein mab-21-like 3",
  "gene": "UniProtKB:Q8N8X9",
  "gene_symbol": "MAB21L3",
  "term_label": "Unknown molecular function",
  "term_id": "UNKNOWN:0001"
}